{
  "term_id": "GO:0031398",
  "gene_name": "Baculoviral IAP repeat-containing protein 8",
  "gene_symbol": "BIRC8",
  "gene": "UniProtKB:Q96P09",
  "term_label": "positive regulation of protein ubiquitination"
}